dIMP salvage [GO:0106385] (biological process) Definition: Any process which produces a dIMP from derivatives of it, without de novo synthesis. References: PMID:8692979 Relationships: is a type of GO:0009171; is_a purine deoxyribonucleotide salvage [GO:0106381]